{
  "gene": "UniProtKB:P57771",
  "gene_name": "Regulator of G-protein signaling 8",
  "gene_symbol": "RGS8",
  "term_id": "GO:0009898",
  "term_label": "cytoplasmic side of plasma membrane"
}